{
  "gene_symbol": "KRT28",
  "term_label": "cytoskeleton",
  "gene": "UniProtKB:Q7Z3Y7",
  "gene_name": "Keratin, type I cytoskeletal 28",
  "term_id": "GO:0005856"
}